regulation of antigen processing and presentation of peptide or polysaccharide antigen via MHC class II [GO:0002580] (biological process) Relationships: is a type of regulation of antigen processing and presentation [GO:0002577]; regulates antigen processing and presentation of peptide or polysaccharide antigen via MHC class II [GO:0002504] Subtypes: negative regulation of antigen processing and presentation of peptide or polysaccharide antigen via MHC class II [GO:0002581], positive regulation of antigen processing and presentation of peptide or polysaccharide antigen via MHC class II [GO:0002582], regulation of antigen processing and presentation of peptide antigen via MHC class II [GO:0002586], regulation of antigen processing and presentation of polysaccharide antigen via MHC class II [GO:0002601] Definition: Any process that modulates the frequency, rate, or extent of antigen processing and presentation of antigen (peptide or polysaccharide) via MHC class II. Sources: GOC:add Also known as: regulation of peptide or polysaccharide antigen processing and presentation via MHC class II